{
  "gene_symbol": "MR1",
  "term_id": "UNKNOWN:0001",
  "gene": "UniProtKB:Q95460",
  "term_label": "Unknown molecular function",
  "gene_name": "Major histocompatibility complex class I-related gene protein"
}